{
  "term_id": "GO:0043434",
  "term_label": "response to peptide hormone",
  "gene_name": "Lithostathine-1-alpha",
  "gene_symbol": "REG1A",
  "gene": "UniProtKB:P05451"
}